{
  "term_label": "Unknown biological process",
  "gene_name": "Trichohyalin-like protein 1",
  "gene": "UniProtKB:Q5QJ38",
  "gene_symbol": "TCHHL1",
  "term_id": "UNKNOWN:0002"
}